{
  "term_label": "signaling receptor binding",
  "gene_symbol": "BTN3A2",
  "gene": "UniProtKB:P78410",
  "term_id": "GO:0005102",
  "gene_name": "Butyrophilin subfamily 3 member A2"
}